ventricular cardiac muscle cell differentiation [GO:0055012] (BP) Sources: GOC:devbiol, GOC:mtg_heart Definition: The process in which a relatively unspecialized cell acquires specialized features of a ventricular cardiac muscle cell. Cardiac muscle cells are striated muscle cells that are responsible for heart contraction. The ventricle is the part of the heart that pumps blood out of the organ. Relationships: is a type of GO:0055007 Also known as: ventricular cardiomyocyte differentiation, ventricular heart muscle cell differentiation